zeaxanthin bis(beta-D-glucoside) catabolic process [GO:1901829] (biological process) Definition: The chemical reactions and pathways resulting in the breakdown of zeaxanthin bis(beta-D-glucoside). References: PMID:20075616 Sources: GOC:TermGenie, GOC:yaf, MetaCyc:PWY-6288, UniPathway:UPA00798 Also known as: zeaxanthin bis(beta-D-glucoside) breakdown, zeaxanthin bis(beta-D-glucoside) catabolism, zeaxanthin bis(beta-D-glucoside) degradation, zeaxanthin diglucoside breakdown, zeaxanthin diglucoside catabolism, zeaxanthin diglucoside degradation Relationships: is a type of carotenoid catabolic process [GO:0016118]; is a type of beta-glucoside catabolic process [GO:1901805]